{
  "term_id": "GO:0016538",
  "gene": "UniProtKB:P24863",
  "gene_symbol": "CCNC",
  "term_label": "cyclin-dependent protein serine/threonine kinase regulator activity",
  "gene_name": "Cyclin-C"
}